cyclin A2-CDK2 complex [GO:0097124] (cellular component) Relationships: is_a cyclin-dependent protein kinase holoenzyme complex [GO:0000307] Definition: A protein complex consisting of cyclin A2 and cyclin-dependent kinase 2 (CDK2). Cyclins are characterized by periodicity in protein abundance throughout the cell cycle. Cyclin-dependent kinases represent a family of serine/threonine protein kinases that become active upon binding to a cyclin regulatory partner. References: PMID:15935619 Sources: GOC:so